{
  "gene_name": "Coiled-coil domain-containing protein 144A",
  "gene": "UniProtKB:A2RUR9",
  "term_id": "UNKNOWN:0002",
  "gene_symbol": "CCDC144A",
  "term_label": "Unknown biological process"
}